detection of other organism [GO:0098543] (biological process) Sources: GOC:dos Definition: The series of events in which a stimulus from another organism is received and converted into a molecular signal. Also known as: recognition of other organism during symbiotic interaction, recognition of other organism involved in symbiotic interaction Subtypes: detection of protozoan [GO:0001563], GO:0002231, detection of nematode [GO:0009600], detection of insect [GO:0009601], detection of symbiont [GO:0009602], detection of bacterium [GO:0016045], detection of fungus [GO:0016046] Relationships: is a type of response to other organism [GO:0051707]; is a type of detection of external biotic stimulus [GO:0098581]